{
  "term_label": "Unknown cellular component",
  "gene_name": "Disintegrin and metalloproteinase domain-containing protein 8",
  "term_id": "UNKNOWN:0003",
  "gene_symbol": "ADAM8",
  "gene": "UniProtKB:P78325"
}